achromobactin transmembrane transporter activity [GO:0042934] (molecular function) Definition: Enables the transfer of achromobactin, a citrate siderophore, from one side of a membrane to the other. Relationships: is a type of siderophore-iron transmembrane transporter activity [GO:0015343]; is a type of GO:0042887; is a type of carboxylic acid transmembrane transporter activity [GO:0046943]; is part of achromobactin transport [GO:0042935] Sources: GOC:jl Also known as: achromobactin transporter activity